{
  "term_label": "olfactory receptor activity",
  "gene_name": "Olfactory receptor 51F2",
  "gene": "UniProtKB:Q8NH61",
  "term_id": "GO:0004984",
  "gene_symbol": "OR51F2"
}